calcium-dependent protein kinase regulator activity [GO:0010858] (molecular function) Relationships: is a type of GO:0019887; regulates calcium-dependent protein serine/threonine kinase activity [GO:0009931] Sources: GOC:dph, GOC:tb Subtypes: calcium-dependent protein kinase inhibitor activity [GO:0008427] Definition: Modulates the activity of a calcium-dependent protein kinase, an enzyme which phosphorylates a protein in a calcium-dependent manner.